positive regulation of bone trabecula formation [GO:1900156] (biological process) Sources: GOC:BHF, GOC:TermGenie Relationships: is a type of positive regulation of developmental process [GO:0051094]; is a type of regulation of bone trabecula formation [GO:1900154]; positively regulates bone trabecula formation [GO:0060346] Also known as: positive regulation of bone trabeculation, positive regulation of skeletal trabecula formation, positive regulation of skeletal trabeculation, up regulation of bone trabecula formation, up regulation of bone trabeculation, up regulation of skeletal trabecula formation, up regulation of skeletal trabeculation, up-regulation of bone trabecula formation, up-regulation of bone trabeculation, up-regulation of skeletal trabecula formation, up-regulation of skeletal trabeculation, upregulation of bone trabecula formation, upregulation of bone trabeculation, upregulation of skeletal trabecula formation, upregulation of skeletal trabeculation, activation of bone trabecula formation, activation of bone trabeculation, activation of skeletal trabecula formation, activation of skeletal trabeculation, activation of bone trabecula biogenesis, activation of skeletal trabecula biogenesis, positive regulation of bone trabecula biogenesis, positive regulation of skeletal trabecula biogenesis, up regulation of bone trabecula biogenesis, up regulation of skeletal trabecula biogenesis, up-regulation of bone trabecula biogenesis, up-regulation of skeletal trabecula biogenesis, upregulation of bone trabecula biogenesis, upregulation of skeletal trabecula biogenesis Definition: Any process that activates or increases the frequency, rate or extent of bone trabecula formation.